{
  "gene_name": "C-C motif chemokine 25",
  "gene_symbol": "CCL25",
  "gene": "UniProtKB:O15444",
  "term_id": "GO:0048020",
  "term_label": "CCR chemokine receptor binding"
}